{
  "term_label": "extracellular matrix organization",
  "gene_symbol": "MMP10",
  "gene_name": "Stromelysin-2",
  "gene": "UniProtKB:P09238",
  "term_id": "GO:0030198"
}